{
  "term_id": "GO:0002323",
  "gene_symbol": "IFNA2",
  "gene": "UniProtKB:P01563",
  "gene_name": "Interferon alpha-2",
  "term_label": "natural killer cell activation involved in immune response"
}